{
  "term_label": "ESCRT III complex",
  "gene_name": "Charged multivesicular body protein 2a",
  "gene": "UniProtKB:O43633",
  "term_id": "GO:0000815",
  "gene_symbol": "CHMP2A"
}